{
  "term_id": "UNKNOWN:0003",
  "gene_symbol": "TRAJ10",
  "gene_name": "Possible J 10 gene (Fragment)",
  "gene": "UniProtKB:A0N4Z7",
  "term_label": "Unknown cellular component"
}